{
  "term_id": "GO:0043491",
  "term_label": "phosphatidylinositol 3-kinase/protein kinase B signal transduction",
  "gene_name": "Unconventional myosin-XVI",
  "gene_symbol": "MYO16",
  "gene": "UniProtKB:Q9Y6X6"
}